{
  "gene": "UniProtKB:Q15311",
  "term_label": "small GTPase-mediated signal transduction",
  "gene_name": "RalA-binding protein 1",
  "gene_symbol": "RALBP1",
  "term_id": "GO:0007264"
}